{
  "term_label": "cysteine-type endopeptidase activator activity",
  "gene_name": "NACHT, LRR and PYD domains-containing protein 1",
  "gene": "UniProtKB:Q9C000",
  "gene_symbol": "NLRP1",
  "term_id": "GO:0140608"
}